positive regulation of mast cell chemotaxis [GO:0060754] (biological process) Sources: GOC:dph, GOC:tb Relationships: is a type of positive regulation of leukocyte chemotaxis [GO:0002690]; is_a regulation of mast cell chemotaxis [GO:0060753]; positively regulates mast cell chemotaxis [GO:0002551] Definition: Any process that increases the rate, frequency or extent of mast cell chemotaxis. Mast cell chemotaxis is the movement of a mast cell in response to an external stimulus.